{
  "gene": "UniProtKB:P54259",
  "term_label": "transcription corepressor activity",
  "gene_symbol": "ATN1",
  "term_id": "GO:0003714",
  "gene_name": "Atrophin-1"
}